{
  "gene_name": "High affinity immunoglobulin epsilon receptor subunit beta",
  "gene_symbol": "MS4A2",
  "term_label": "plasma membrane",
  "gene": "UniProtKB:Q01362",
  "term_id": "GO:0005886"
}